{
  "gene_symbol": "GLE1",
  "term_label": "translation initiation factor binding",
  "gene_name": "mRNA export factor GLE1",
  "term_id": "GO:0031369",
  "gene": "UniProtKB:Q53GS7"
}